{
  "gene": "UniProtKB:Q8NFD4",
  "term_id": "UNKNOWN:0002",
  "term_label": "Unknown biological process",
  "gene_symbol": "Q8NFD4",
  "gene_name": "Uncharacterized protein FLJ76381"
}